post-translational protein targeting to endoplasmic reticulum membrane [GO:0006620] (biological process) Relationships: is_a protein targeting to membrane [GO:0006612]; is a type of protein targeting to ER [GO:0045047] Definition: The targeting of proteins to a membrane that occurs after their translation. Some secretory proteins exhibit posttranslational transport into the endoplasmic reticulum (ER) lumen: they are synthesized in their entirety on free cytosolic ribosomes and then released into the cytosol, where they are bound by chaperones which keep them in an unfolded state, and subsequently are translocated across the ER membrane. Sources: ISBN:0716731363 Also known as: SRP-independent endoplasmic reticulum protein-membrane targeting, posttranslational endoplasmic reticulum membrane targeting, posttranslational endoplasmic reticulum protein-membrane targeting, posttranslational protein endoplasmic reticulum membrane targeting, posttranslational protein targeting to ER membrane, posttranslational protein targeting to endoplasmic reticulum membrane